purine-specific mismatch base pair DNA N-glycosylase activity [GO:0000701] (molecular function) Relationships: is a type of mismatch base pair DNA N-glycosylase activity [GO:0000700] References: PMID:9224623 Sources: GOC:elh Definition: Catalysis of the removal of purines present in mismatches, especially opposite oxidized purines, by cleaving the N-C1' glycosidic bond between the target damaged DNA base and the deoxyribose sugar. The reaction releases a free base and leaves an apurinic (AP) site. Also known as: A/G-specific adenine DNA glycosylase activity